{
  "gene": "UniProtKB:O15260",
  "gene_symbol": "SURF4",
  "term_id": "GO:0007030",
  "term_label": "Golgi organization",
  "gene_name": "Surfeit locus protein 4"
}